{
  "gene": "UniProtKB:P09104",
  "gene_symbol": "ENO2",
  "gene_name": "Gamma-enolase",
  "term_label": "phosphopyruvate hydratase activity",
  "term_id": "GO:0004634"
}